{
  "term_label": "negative regulation of transcription by RNA polymerase II",
  "gene_symbol": "CABIN1",
  "term_id": "GO:0000122",
  "gene_name": "Calcineurin-binding protein cabin-1",
  "gene": "UniProtKB:Q9Y6J0"
}